{
  "gene_name": "Glutamate receptor ionotropic, kainate 3",
  "gene": "UniProtKB:Q13003",
  "gene_symbol": "GRIK3",
  "term_label": "presynaptic membrane",
  "term_id": "GO:0042734"
}